{
  "term_label": "Unknown molecular function",
  "gene": "UniProtKB:Q6ZP68",
  "term_id": "UNKNOWN:0001",
  "gene_symbol": "ATP11AUN",
  "gene_name": "Putative protein ATP11AUN"
}